{
  "term_id": "UNKNOWN:0003",
  "gene": "UniProtKB:Q8N9M5",
  "term_label": "Unknown cellular component",
  "gene_symbol": "TMEM102",
  "gene_name": "Transmembrane protein 102"
}